{
  "term_id": "UNKNOWN:0002",
  "gene": "UniProtKB:Q6U949",
  "term_label": "Unknown biological process",
  "gene_symbol": "IGF2-AS",
  "gene_name": "Putative insulin-like growth factor 2 antisense gene protein"
}